{
  "term_label": "endoplasmic reticulum membrane",
  "gene_symbol": "ABHD12",
  "term_id": "GO:0005789",
  "gene_name": "Lysophosphatidylserine lipase ABHD12",
  "gene": "UniProtKB:Q8N2K0"
}